{
  "gene_name": "Putative uncharacterized protein KTN1-AS1",
  "term_label": "Unknown cellular component",
  "gene": "UniProtKB:Q86SY8",
  "gene_symbol": "KTN1-AS1",
  "term_id": "UNKNOWN:0003"
}